{
  "gene_symbol": "TSC2",
  "term_label": "GTPase activator activity",
  "gene": "UniProtKB:P49815",
  "gene_name": "Tuberin",
  "term_id": "GO:0005096"
}